{
  "gene": "UniProtKB:A0A075B6U8",
  "term_id": "UNKNOWN:0001",
  "gene_symbol": "TRAJ12",
  "term_label": "Unknown molecular function",
  "gene_name": "T cell receptor alpha joining 12 (Fragment)"
}